{
  "term_id": "GO:0000977",
  "term_label": "RNA polymerase II transcription regulatory region sequence-specific DNA binding",
  "gene_symbol": "ASCL5",
  "gene_name": "Achaete-scute homolog 5",
  "gene": "UniProtKB:Q7RTU5"
}